{
  "gene_symbol": "C3orf85",
  "gene": "UniProtKB:A0A1B0GTC6",
  "term_id": "UNKNOWN:0002",
  "gene_name": "Uncharacterized protein C3orf85",
  "term_label": "Unknown biological process"
}